{
  "term_id": "UNKNOWN:0002",
  "gene_name": "ProSAAS",
  "gene_symbol": "PCSK1N",
  "gene": "UniProtKB:Q9UHG2",
  "term_label": "Unknown biological process"
}